ATPase binding [GO:0051117] (molecular function) Definition: Binding to an ATPase, any enzyme that catalyzes the hydrolysis of ATP. Relationships: is a type of enzyme binding [GO:0019899] Sources: GOC:ai